{
  "gene": "UniProtKB:P63000",
  "term_id": "GO:0030031",
  "gene_name": "Ras-related C3 botulinum toxin substrate 1",
  "term_label": "cell projection assembly",
  "gene_symbol": "RAC1"
}